{
  "gene_name": "BTB_POZ domain-containing protein 2",
  "gene_symbol": "BTBD2",
  "term_label": "P-body",
  "gene": "UniProtKB:Q9BX70",
  "term_id": "GO:0000932"
}